{
  "gene_name": "Nucleolar protein 9",
  "term_label": "90S preribosome",
  "gene": "UniProtKB:Q86U38",
  "term_id": "GO:0030686",
  "gene_symbol": "NOP9"
}